elaioplast stroma [GO:0009577] (cellular component) Relationships: is a type of GO:0009532; is part of elaioplast [GO:0009545] Definition: The space enclosed by the double membrane of an elaioplast. Sources: GOC:mah